{
  "gene_symbol": "CD163L1",
  "gene_name": "Scavenger receptor cysteine-rich type 1 protein M160",
  "gene": "UniProtKB:Q9NR16",
  "term_label": "scavenger receptor activity",
  "term_id": "GO:0005044"
}